{
  "gene_symbol": "NRG4",
  "term_id": "UNKNOWN:0003",
  "term_label": "Unknown cellular component",
  "gene_name": "Pro-neuregulin-4, membrane-bound isoform",
  "gene": "UniProtKB:Q8WWG1"
}